leukocyte migration [GO:0050900] (biological process) Also known as: immune cell migration, immune cell trafficking, leucocyte migration, leucocyte trafficking, leukocyte trafficking Relationships: is a type of immune system process [GO:0002376]; is a type of cell migration [GO:0016477] Definition: The movement of a leukocyte within or between different tissues and organs of the body. References: PMID:14680625, PMID:14708592, PMID:7507411, PMID:8600538 Sources: GOC:add, ISBN:0781735149 Subtypes: leukocyte migration involved in immune response [GO:0002522], leukocyte migration involved in inflammatory response [GO:0002523], leukocyte chemotaxis [GO:0030595], cellular extravasation [GO:0045123], diapedesis [GO:0050904], mononuclear cell migration [GO:0071674], GO:0097529 Regulation: regulated by regulation of leukocyte migration [GO:0002685]; negatively regulated by GO:0002686; positively regulated by GO:0002687